{
  "gene": "UniProtKB:P0CG39",
  "gene_symbol": "POTEJ",
  "term_label": "axonogenesis",
  "term_id": "GO:0007409",
  "gene_name": "POTE ankyrin domain family member J"
}